{
  "gene_symbol": "AP1S2",
  "gene": "UniProtKB:P56377",
  "term_label": "Unknown cellular component",
  "term_id": "UNKNOWN:0003",
  "gene_name": "AP-1 complex subunit sigma-2"
}